{
  "gene_symbol": "ENDOG",
  "gene": "UniProtKB:Q14249",
  "term_id": "GO:0000014",
  "term_label": "single-stranded DNA endodeoxyribonuclease activity",
  "gene_name": "Endonuclease G, mitochondrial"
}